{
  "term_id": "GO:0005901",
  "gene": "UniProtKB:Q8WTV0",
  "term_label": "caveola",
  "gene_symbol": "SCARB1",
  "gene_name": "Scavenger receptor class B member 1"
}